regulation of tatiopterin biosynthetic process [GO:1900974] (biological process) Also known as: regulation of tatiopterin anabolism, regulation of tatiopterin biosynthesis, regulation of tatiopterin formation, regulation of tatiopterin synthesis Subtypes: negative regulation of tatiopterin biosynthetic process [GO:1900975], GO:1900976 Sources: GOC:TermGenie, GOC:mengo_curators Relationships: is_a regulation of biosynthetic process [GO:0009889]; is a type of GO:0051174; is a type of regulation of small molecule metabolic process [GO:0062012]; regulates GO:1900870 Definition: Any process that modulates the frequency, rate or extent of tatiopterin biosynthetic process.